L-arginine catabolic process to L-glutamate [GO:0019544] (biological process) Sources: GOC:go_curators Also known as: arginine breakdown to glutamate, arginine degradation to glutamate Relationships: is a type of GO:0006527; is_a GO:0006536 Definition: The chemical reactions and pathways resulting in the breakdown of L-arginine into other compounds, including L-glutamate.